{
  "gene_name": "Spermatogenesis-associated protein 2",
  "gene_symbol": "SPATA2",
  "term_label": "regulation of necroptotic process",
  "term_id": "GO:0060544",
  "gene": "UniProtKB:Q9UM82"
}